{
  "gene_symbol": "ABCD1",
  "term_id": "GO:0006635",
  "term_label": "fatty acid beta-oxidation",
  "gene": "UniProtKB:P33897",
  "gene_name": "ATP-binding cassette sub-family D member 1"
}